{
  "gene_symbol": "ZNF555",
  "gene": "UniProtKB:Q8NEP9",
  "term_label": "DNA-binding transcription factor activity, RNA polymerase II-specific",
  "gene_name": "Zinc finger protein 555",
  "term_id": "GO:0000981"
}